conoid [GO:0020010] (cellular component) References: PMID:11901169, PMID:16518471 Sources: GOC:expert_dr Definition: A spiral cytoskeletal structure located at the apical end of the apical complex in some apicomplexan parasites. Fibers form a left-handed spiral, and are comprised of tubulin protofilaments organized in a ribbon-like structure that differs from the conventional tubular structure characteristic of microtubules. Relationships: is_a GO:0110165; is part of GO:0005856; is part of apical complex [GO:0020007]